{
  "term_label": "Unknown molecular function",
  "term_id": "UNKNOWN:0001",
  "gene": "UniProtKB:Q52LA3",
  "gene_symbol": "LIN52",
  "gene_name": "Protein lin-52 homolog"
}